regulation of epithelial to mesenchymal transition [GO:0010717] (BP) Definition: Any process that modulates the rate, frequency, or extent of epithelial to mesenchymal transition. Epithelial to mesenchymal transition where an epithelial cell loses apical/basolateral polarity, severs intercellular adhesive junctions, degrades basement membrane components and becomes a migratory mesenchymal cell. Sources: GOC:BHF, GOC:dph, GOC:tb Relationships: is a type of GO:0045595; regulates epithelial to mesenchymal transition [GO:0001837] Subtypes: GO:0010718, negative regulation of epithelial to mesenchymal transition [GO:0010719], GO:0062042, regulation of neural crest formation [GO:0090299]